{
  "term_label": "ubiquitin conjugating enzyme binding",
  "gene_name": "E3 ubiquitin-protein ligase MARCHF7",
  "term_id": "GO:0031624",
  "gene": "UniProtKB:Q9H992",
  "gene_symbol": "MARCHF7"
}